{
  "gene": "UniProtKB:Q5T0F9",
  "term_id": "GO:0006357",
  "gene_name": "Coiled-coil and C2 domain-containing protein 1B",
  "term_label": "regulation of transcription by RNA polymerase II",
  "gene_symbol": "CC2D1B"
}